{
  "gene": "UniProtKB:Q9ULE0",
  "gene_name": "Protein WWC3",
  "term_id": "GO:0019900",
  "gene_symbol": "WWC3",
  "term_label": "kinase binding"
}